epithelial cell proliferation involved in mammary gland bud elongation [GO:0060650] (biological process) Regulation: regulated by GO:0060651 References: PMID:12558599 Sources: GOC:dph Definition: The multiplication or reproduction of mammary gland bud epithelial cells, resulting in the elongation of the bud. Relationships: is a type of GO:0033598; is part of mammary gland bud elongation [GO:0060649]